{
  "gene_name": "Zinc finger protein 397",
  "gene_symbol": "ZNF397",
  "term_id": "GO:0000978",
  "term_label": "RNA polymerase II cis-regulatory region sequence-specific DNA binding",
  "gene": "UniProtKB:Q8NF99"
}